{
  "term_label": "Unknown cellular component",
  "gene_name": "Immunoglobulin heavy variable 4-28",
  "term_id": "UNKNOWN:0003",
  "gene_symbol": "IGHV4-28",
  "gene": "UniProtKB:A0A0C4DH34"
}